cellular response to trichostatin A [GO:0035984] (biological process) Definition: Any process that results in a change in state or activity of a cell (in terms of movement, secretion, enzyme production, gene expression, etc.) as a result of a trichostatin A stimulus. Relationships: is a type of response to trichostatin A [GO:0035983]; is a type of cellular response to antibiotic [GO:0071236]; is_a cellular response to nitrogen compound [GO:1901699]; is a type of cellular response to oxygen-containing compound [GO:1901701] References: PMID:20181743 Sources: GOC:yaf